{
  "gene_name": "Small integral membrane protein 40",
  "term_label": "Unknown molecular function",
  "gene_symbol": "SMIM40",
  "gene": "UniProtKB:Q5STR5",
  "term_id": "UNKNOWN:0001"
}